regulation of growth of unicellular organism as a thread of attached cells [GO:0070784] (biological process) Relationships: is a type of GO:1900428; regulates growth of unicellular organism as a thread of attached cells [GO:0070783] Definition: Any process that modulates the frequency, rate or extent of the process in which cells remain attached after division and form thread-like filaments that may penetrate into a solid growth medium. Subtypes: cell growth mode switching, budding to filamentous [GO:0036187], negative regulation of growth of unicellular organism as a thread of attached cells [GO:0070785], positive regulation of growth of unicellular organism as a thread of attached cells [GO:0070786], GO:0097321, regulation of invasive growth in response to glucose limitation [GO:2000217], regulation of pseudohyphal growth [GO:2000220] Sources: GOC:mah